nitric oxide dioxygenase NAD(P)H activity [GO:0008941] (MF) Sources: EC:1.14.12.17 Also known as: nitric oxide dioxygenase activity, NOD activity Definition: Catalysis of the reaction: 2 NO + 2 O2 + NAD(P)H + H+ = 2 nitrate + NAD(P)+. Note: Note that this activity is similar to nitric oxide dioxygenase activity, heme protein ; GO:0141118, but GO:0141118 uses a heme protein as the electron donor. Relationships: is_a oxidoreductase activity, acting on paired donors, with incorporation or reduction of molecular oxygen, NAD(P)H as one donor, and incorporation of two atoms of oxygen into one donor [GO:0016708]